{
  "gene_symbol": "NEUROG1",
  "term_id": "GO:0030900",
  "gene_name": "Neurogenin-1",
  "term_label": "forebrain development",
  "gene": "UniProtKB:Q92886"
}